{
  "gene_name": "Fumarylacetoacetase",
  "gene_symbol": "FAH",
  "term_id": "GO:0004334",
  "gene": "UniProtKB:P16930",
  "term_label": "fumarylacetoacetase activity"
}